{
  "gene_symbol": "TRAV8-6",
  "gene_name": "T cell receptor alpha variable 8-6",
  "term_label": "immunoglobulin complex",
  "gene": "UniProtKB:A0A0B4J262",
  "term_id": "GO:0019814"
}